{
  "gene_name": "Small integral membrane protein 5",
  "term_label": "Unknown cellular component",
  "term_id": "UNKNOWN:0003",
  "gene_symbol": "SMIM5",
  "gene": "UniProtKB:Q71RC9"
}